{
  "term_id": "GO:0030674",
  "term_label": "protein-macromolecule adaptor activity",
  "gene": "UniProtKB:Q15811",
  "gene_symbol": "ITSN1",
  "gene_name": "Intersectin-1"
}